{
  "gene_symbol": "CEP164",
  "gene": "UniProtKB:Q9UPV0",
  "term_label": "ciliary transition fiber",
  "gene_name": "Centrosomal protein of 164 kDa",
  "term_id": "GO:0097539"
}